{
  "gene": "UniProtKB:Q8NEC5",
  "gene_symbol": "CATSPER1",
  "term_label": "calcium ion transport",
  "gene_name": "Cation channel sperm-associated protein 1",
  "term_id": "GO:0006816"
}